{
  "gene_symbol": "RPH3AL",
  "gene": "UniProtKB:Q9UNE2",
  "gene_name": "Rab effector Noc2",
  "term_label": "calcium-dependent activation of synaptic vesicle fusion",
  "term_id": "GO:0099502"
}